positive regulation of corticotropin-releasing hormone secretion [GO:0051466] (biological process) Sources: GOC:ai Relationships: is a type of regulation of corticotropin-releasing hormone secretion [GO:0043397]; is a type of GO:0090277; positively regulates corticotropin-releasing hormone secretion [GO:0043396] Also known as: positive regulation of CRF secretion, positive regulation of CRH secretion, positive regulation of corticotropin-releasing factor secretion, up regulation of corticotropin-releasing hormone secretion, up-regulation of corticotropin-releasing hormone secretion, upregulation of corticotropin-releasing hormone secretion, activation of corticotropin-releasing hormone secretion, stimulation of corticotropin-releasing hormone secretion Definition: Any process that activates or increases the frequency, rate or extent of the regulated release of corticotropin-releasing hormone from a cell.